{
  "gene": "UniProtKB:A0A075B6Z1",
  "gene_symbol": "TRAJ20",
  "gene_name": "T cell receptor alpha joining 20 (Fragment)",
  "term_label": "Unknown cellular component",
  "term_id": "UNKNOWN:0003"
}